{
  "gene_name": "Notch homolog 2 N-terminal-like protein B",
  "gene": "UniProtKB:P0DPK3",
  "gene_symbol": "NOTCH2NLB",
  "term_id": "UNKNOWN:0003",
  "term_label": "Unknown cellular component"
}